{
  "term_label": "Unknown cellular component",
  "term_id": "UNKNOWN:0003",
  "gene_symbol": "KBTBD11",
  "gene_name": "Kelch repeat and BTB domain-containing protein 11",
  "gene": "UniProtKB:O94819"
}